{
  "term_id": "UNKNOWN:0001",
  "gene_name": "Vitamin K-dependent protein S",
  "gene_symbol": "PROS1",
  "term_label": "Unknown molecular function",
  "gene": "UniProtKB:P07225"
}